phosphatidylserine biosynthetic process [GO:0006659] (biological process) Regulation: regulated by regulation of phosphatidylserine biosynthetic process [GO:1900468]; negatively regulated by GO:1900469; positively regulated by positive regulation of phosphatidylserine biosynthetic process [GO:1900470] Relationships: is a type of phosphatidylserine metabolic process [GO:0006658]; is a type of modified amino acid biosynthetic process [GO:0042398]; is a type of GO:0046474 Also known as: phosphatidylserine anabolism, phosphatidylserine biosynthesis, phosphatidylserine formation, phosphatidylserine synthesis Sources: ISBN:0198506732 Definition: The chemical reactions and pathways resulting in the formation of phosphatidylserines, any of a class of glycerophospholipids in which the phosphatidyl group is esterified to the hydroxyl group of L-serine.